regulation of toll-like receptor 9 signaling pathway [GO:0034163] (biological process) Relationships: is_a regulation of cytoplasmic pattern recognition receptor signaling pathway [GO:0039531]; regulates toll-like receptor 9 signaling pathway [GO:0034162] Also known as: regulation of TLR9 signaling pathway, regulation of toll-like receptor 9 signalling pathway Subtypes: GO:0034164, positive regulation of toll-like receptor 9 signaling pathway [GO:0034165] References: PMID:16551253, PMID:17328678 Sources: GOC:add Definition: Any process that modulates the frequency, rate, or extent of toll-like receptor 9 signaling pathway.